{
  "gene_name": "Serine_threonine-protein kinase pim-2",
  "gene": "UniProtKB:Q9P1W9",
  "term_id": "GO:0043123",
  "term_label": "positive regulation of canonical NF-kappaB signal transduction",
  "gene_symbol": "PIM2"
}